{
  "term_label": "signaling receptor binding",
  "gene_symbol": "FYN",
  "gene_name": "Tyrosine-protein kinase Fyn",
  "gene": "UniProtKB:P06241",
  "term_id": "GO:0005102"
}